{
  "term_id": "UNKNOWN:0002",
  "gene": "UniProtKB:Q8WZ94",
  "term_label": "Unknown biological process",
  "gene_symbol": "OR5P3",
  "gene_name": "Olfactory receptor 5P3"
}